{
  "term_id": "GO:0016616",
  "term_label": "oxidoreductase activity, acting on the CH-OH group of donors, NAD or NADP as acceptor",
  "gene_name": "3 beta-hydroxysteroid dehydrogenase type 7",
  "gene": "UniProtKB:Q9H2F3",
  "gene_symbol": "HSD3B7"
}